negative regulation of platelet-derived growth factor receptor signaling pathway [GO:0010642] (biological process) Relationships: is a type of negative regulation of signal transduction [GO:0009968]; is a type of regulation of platelet-derived growth factor receptor signaling pathway [GO:0010640]; negatively regulates GO:0048008 Definition: Any process that stops, prevents, or reduces the frequency, rate or extent of the platelet-derived growth factor receptor signaling pathway. Also known as: negative regulation of platelet-derived growth factor receptor signalling pathway Subtypes: negative regulation of platelet-derived growth factor receptor-alpha signaling pathway [GO:2000584], negative regulation of platelet-derived growth factor receptor-beta signaling pathway [GO:2000587] Sources: GOC:dph, GOC:hjd, GOC:tb